{
  "gene_name": "Kallikrein-13",
  "term_label": "protein maturation",
  "gene": "UniProtKB:Q9UKR3",
  "gene_symbol": "KLK13",
  "term_id": "GO:0051604"
}